{
  "gene_symbol": "CLEC2B",
  "term_id": "GO:0005886",
  "gene_name": "C-type lectin domain family 2 member B",
  "gene": "UniProtKB:Q92478",
  "term_label": "plasma membrane"
}